{
  "term_id": "GO:0008236",
  "term_label": "serine-type peptidase activity",
  "gene_name": "Transmembrane protease serine 12",
  "gene_symbol": "TMPRSS12",
  "gene": "UniProtKB:Q86WS5"
}